{
  "term_id": "GO:0005912",
  "gene_name": "LIM domain-containing protein ajuba",
  "gene": "UniProtKB:Q96IF1",
  "gene_symbol": "AJUBA",
  "term_label": "adherens junction"
}